acinar cell proliferation [GO:1990863] (biological process) Also known as: acinic cell proliferation, acinous cell proliferation Regulation: regulated by regulation of acinar cell proliferation [GO:1904697]; negatively regulated by negative regulation of acinar cell proliferation [GO:1904698]; positively regulated by positive regulation of acinar cell proliferation [GO:1904699] Relationships: is a type of epithelial cell proliferation [GO:0050673] Definition: The multiplication or reproduction of acinar cells, resulting in the expansion of a cell population. An acinar cell is a secretory cell that is grouped together with other cells of the same type to form grape-shaped clusters known as acini (singular acinus). References: PMID:9788538